{
  "gene_symbol": "FAM83H",
  "gene_name": "Protein FAM83H",
  "term_id": "GO:1990254",
  "gene": "UniProtKB:Q6ZRV2",
  "term_label": "keratin filament binding"
}